cellular response to superoxide [GO:0071451] (biological process) Relationships: is a type of response to superoxide [GO:0000303]; is_a GO:0071450 Definition: Any process that results in a change in state or activity of a cell (in terms of movement, secretion, enzyme production, gene expression, etc.) as a result of a superoxide stimulus. Superoxide is the anion, oxygen-, formed by addition of one electron to dioxygen (O2) or any compound containing the superoxide anion. Sources: GOC:mah